positive regulation of granulocyte differentiation [GO:0030854] (BP) Sources: GOC:mah Relationships: is a type of positive regulation of myeloid leukocyte differentiation [GO:0002763]; is a type of GO:0030852; positively regulates granulocyte differentiation [GO:0030851] Definition: Any process that activates or increases the frequency, rate or extent of granulocyte differentiation. Subtypes: positive regulation of basophil differentiation [GO:0045642], positive regulation of eosinophil differentiation [GO:0045645], positive regulation of neutrophil differentiation [GO:0045660] Also known as: up regulation of granulocyte differentiation, up-regulation of granulocyte differentiation, upregulation of granulocyte differentiation, activation of granulocyte differentiation, stimulation of granulocyte differentiation